juxtaglomerulus cell differentiation [GO:0072052] (biological process) Sources: GOC:mtg_kidney_jan10 Subtypes: mesonephric juxtaglomerulus cell differentiation [GO:0061207], metanephric juxtaglomerulus cell differentiation [GO:0072251] Relationships: is a type of cell differentiation involved in kidney development [GO:0061005]; is part of GO:0072051 Definition: The process in which relatively unspecialized cells acquire specialized structural and/or functional features that characterize the juxtaglomerulus cells of the kidney as it progresses from its formation to the mature state.